bacteriochlorophyll biosynthetic process [GO:0030494] (biological process) Definition: The chemical reactions and pathways resulting in the formation of a bacteriochlorophyll, any of the chlorophylls of photosynthetic bacteria. They differ structurally from the chlorophylls of higher plants. Subtypes: light-dependent bacteriochlorophyll biosynthetic process [GO:0036069], light-independent bacteriochlorophyll biosynthetic process [GO:0036070] Also known as: bacteriochlorophyll anabolism, bacteriochlorophyll biosynthesis, bacteriochlorophyll formation, bacteriochlorophyll synthesis Relationships: is a type of chlorophyll biosynthetic process [GO:0015995] Sources: GOC:mah, ISBN:0198506732